{
  "gene_symbol": "CCL4",
  "gene": "UniProtKB:P13236",
  "gene_name": "C-C motif chemokine 4",
  "term_id": "GO:0005615",
  "term_label": "extracellular space"
}